{
  "term_id": "GO:0007165",
  "gene": "UniProtKB:Q92597",
  "term_label": "signal transduction",
  "gene_name": "Protein NDRG1",
  "gene_symbol": "NDRG1"
}